amino acid neurotransmitter reuptake [GO:0051933] (biological process) Regulation: regulated by regulation of amino acid uptake involved in synaptic transmission [GO:0051941]; negatively regulated by negative regulation of amino acid uptake involved in synaptic transmission [GO:0051942]; positively regulated by positive regulation of amino acid uptake involved in synaptic transmission [GO:0051943] Subtypes: glutamate reuptake [GO:0051935], gamma-aminobutyric acid reuptake [GO:0051936] Definition: The uptake of amino acid neurotransmitters by neurons or glial cells. This process leads to inactivation and recycling of neurotransmitters. Relationships: is a type of amino acid transport [GO:0006865]; is a type of neurotransmitter reuptake [GO:0098810] Also known as: amino acid neurotransmitter recycling, amino acid neurotransmitter import into glial cell, amino acid neurotransmitter import into neuron, amino acid uptake during transmission of nerve impulse Sources: ISBN:0123668387